{
  "term_label": "dipeptidyl-peptidase activity",
  "term_id": "GO:0008239",
  "gene_symbol": "DPP8",
  "gene_name": "Dipeptidyl peptidase 8",
  "gene": "UniProtKB:Q6V1X1"
}